{
  "term_id": "UNKNOWN:0001",
  "gene": "UniProtKB:Q5T7R7",
  "term_label": "Unknown molecular function",
  "gene_symbol": "C1orf185",
  "gene_name": "Uncharacterized protein C1orf185"
}